{
  "gene_symbol": "CENPU",
  "term_label": "Unknown biological process",
  "gene": "UniProtKB:Q71F23",
  "term_id": "UNKNOWN:0002",
  "gene_name": "Centromere protein U"
}